MBF transcription complex [GO:0030907] (cellular component) Definition: A protein complex that binds to the Mlu1 cell cycle box (MCB) promoter element, consensus sequence ACGCGN, and is involved in regulation of transcription during the G1/S transition of the cell cycle. In Saccharomyces, the complex contains a heterodimer of the DNA binding protein Mbp1p and the activator Swi6p, and is associated with additional proteins known as Nrm1p, Msa1p, and Msa2p; in Schizosaccharomyces the complex contains Res1p, Res2p, and Cdc10p. Also known as: DSC1 transcription factor complex, MBF, Mlu1-box binding factor References: PMID:11206552, PMID:15838511, PMID:18160399, PMID:9343385 Sources: GOC:mah Relationships: is a type of RNA polymerase II transcription regulator complex [GO:0090575]